{
  "gene": "UniProtKB:P62979",
  "gene_symbol": "RPS27A",
  "gene_name": "Ubiquitin-ribosomal protein eS31 fusion protein",
  "term_label": "protein ubiquitination",
  "term_id": "GO:0016567"
}